{
  "gene_symbol": "ABCB7",
  "term_label": "ATPase-coupled transmembrane transporter activity",
  "gene_name": "Iron-sulfur clusters transporter ABCB7, mitochondrial",
  "gene": "UniProtKB:O75027",
  "term_id": "GO:0042626"
}